RNA endonuclease activity [GO:0004521] (molecular function) Definition: Catalysis of the cleavage of ester linkages within ribonucleic acid by creating internal breaks. Also known as: endoribonuclease activity, endonuclease G activity Relationships: is a type of endonuclease activity [GO:0004519]; is a type of RNA nuclease activity [GO:0004540] Regulation: negatively regulated by endoribonuclease inhibitor activity [GO:0060698]; regulated by regulation of endoribonuclease activity [GO:0060699]; negatively regulated by GO:0060702 Sources: GOC:mah, ISBN:0198547684 Subtypes: ribonuclease MRP activity [GO:0000171], tRNA-intron lyase activity [GO:0000213], ribonuclease A activity [GO:0004522], Enterobacter ribonuclease activity [GO:0008847], RNA endonuclease activity producing 5'-phosphomonoesters, hydrolytic mechanism [GO:0016891], GO:0016892, GO:0033897, GO:0033899, rRNA endonuclease activity [GO:0033902], GO:0046589